{
  "gene_symbol": "RB1",
  "term_label": "RNA polymerase II transcription regulatory region sequence-specific DNA binding",
  "gene_name": "Retinoblastoma-associated protein",
  "gene": "UniProtKB:P06400",
  "term_id": "GO:0000977"
}